{
  "gene_name": "Metalloproteinase inhibitor 2",
  "term_label": "response to cytokine",
  "term_id": "GO:0034097",
  "gene_symbol": "TIMP2",
  "gene": "UniProtKB:P16035"
}